{
  "gene_symbol": "COMMD1",
  "gene": "UniProtKB:Q8N668",
  "term_id": "GO:0031398",
  "gene_name": "COMM domain-containing protein 1",
  "term_label": "positive regulation of protein ubiquitination"
}